{
  "gene": "UniProtKB:A6NC86",
  "gene_symbol": "PINLYP",
  "term_id": "UNKNOWN:0002",
  "gene_name": "phospholipase A2 inhibitor and Ly6_PLAUR domain-containing protein",
  "term_label": "Unknown biological process"
}